{
  "gene_name": "EH domain-containing protein 2",
  "gene": "UniProtKB:Q9NZN4",
  "term_id": "GO:0032456",
  "gene_symbol": "EHD2",
  "term_label": "endocytic recycling"
}